{
  "gene_symbol": "ADAM21",
  "term_id": "GO:0005886",
  "gene_name": "Disintegrin and metalloproteinase domain-containing protein 21",
  "gene": "UniProtKB:Q9UKJ8",
  "term_label": "plasma membrane"
}